{
  "gene_name": "Putative UPF0607 protein LOC392364",
  "term_id": "UNKNOWN:0001",
  "term_label": "Unknown molecular function",
  "gene_symbol": "Q5PR19",
  "gene": "UniProtKB:Q5PR19"
}